{
  "gene": "UniProtKB:Q86SQ0",
  "gene_name": "Pleckstrin homology-like domain family B member 2",
  "term_id": "GO:0045180",
  "gene_symbol": "PHLDB2",
  "term_label": "basal cortex"
}